{
  "term_id": "GO:0000149",
  "gene_name": "Syntaxin-3",
  "gene_symbol": "STX3",
  "term_label": "SNARE binding",
  "gene": "UniProtKB:Q13277"
}